{
  "gene": "UniProtKB:Q9BRJ9",
  "term_label": "DNA-binding transcription factor activity, RNA polymerase II-specific",
  "gene_symbol": "MESP1",
  "gene_name": "Mesoderm posterior protein 1",
  "term_id": "GO:0000981"
}